inositol-1,2,4,5-tetrakisphosphate 5-phosphatase activity [GO:1990649] (molecular function) Relationships: is a type of inositol tetrakisphosphate phosphatase activity [GO:0052743] Definition: Catalysis of the reaction: 1D-myo-inositol 1,2,4,5-tetrakisphosphate + H2O = 1D-myo-inositol 1,2,4-trisphosphate + phosphate. References: PMID:15316017 Sources: GOC:al